indoleacetic acid biosynthetic process via tryptophan [GO:0009848] (biological process) Regulation: regulated by regulation of indoleacetic acid biosynthetic process via tryptophan [GO:1901996]; negatively regulated by negative regulation of indoleacetic acid biosynthetic process via tryptophan [GO:1901997] Also known as: IAA biosynthetic process via tryptophan, indoleacetic acid anabolism via tryptophan, indoleacetic acid formation via tryptophan, indoleacetic acid synthesis via tryptophan References: PMID:10375566 Sources: GOC:lm, GOC:lr Definition: The chemical reactions and pathways resulting in the formation of indole-3-acetic acid that occurs through metabolism of L-tryptophan. Relationships: is a type of L-tryptophan metabolic process [GO:0006568]; is a type of indoleacetic acid biosynthetic process [GO:0009684]